{
  "gene": "UniProtKB:Q8TBZ3",
  "gene_name": "WD repeat-containing protein 20",
  "term_label": "nucleus",
  "gene_symbol": "WDR20",
  "term_id": "GO:0005634"
}